{
  "gene": "UniProtKB:Q9BYR3",
  "gene_symbol": "KRTAP4-4",
  "gene_name": "Keratin-associated protein 4-4",
  "term_id": "UNKNOWN:0001",
  "term_label": "Unknown molecular function"
}